PAM complex, Tim23 associated import motor [GO:0001405] (cellular component) Definition: Protein complex located on the matrix side of the mitochondrial inner membrane and associated with the TIM23 mitochondrial import inner membrane translocase complex (GO:0005744); ATPase motor activity to drive import of proteins into the mitochondrial matrix. References: PMID:14517234, PMID:14638855 Sources: GOC:mcc, GOC:vw Also known as: PAM complex, mitochondrial import motor, pre-sequence translocase-associated import motor, presequence translocase-associated import motor Relationships: is a type of GO:0098800; is part of TIM23 mitochondrial import inner membrane translocase complex [GO:0005744]; is part of mitochondrial matrix [GO:0005759]